{
  "gene_name": "Probable ATP-dependent RNA helicase DDX53",
  "term_label": "RNA helicase activity",
  "gene_symbol": "DDX53",
  "gene": "UniProtKB:Q86TM3",
  "term_id": "GO:0003724"
}